{
  "term_label": "odorant binding",
  "gene_name": "Olfactory receptor 5M10",
  "term_id": "GO:0005549",
  "gene": "UniProtKB:Q6IEU7",
  "gene_symbol": "OR5M10"
}